{
  "term_label": "DNA-binding transcription factor activity, RNA polymerase II-specific",
  "gene_name": "Zinc finger protein 775",
  "gene_symbol": "ZNF775",
  "term_id": "GO:0000981",
  "gene": "UniProtKB:Q96BV0"
}